{
  "gene": "UniProtKB:P51681",
  "term_id": "GO:0006955",
  "gene_name": "C-C chemokine receptor type 5",
  "gene_symbol": "CCR5",
  "term_label": "immune response"
}